negative regulation of endothelial cell chemotaxis [GO:2001027] (biological process) Subtypes: negative regulation of endothelial cell chemotaxis to fibroblast growth factor [GO:2000545] Definition: Any process that stops, prevents or reduces the frequency, rate or extent of endothelial cell chemotaxis. Relationships: is a type of negative regulation of endothelial cell migration [GO:0010596]; is a type of negative regulation of chemotaxis [GO:0050922]; is a type of GO:2001026; negatively regulates GO:0035767 Sources: GOC:BHF